myosin I binding [GO:0017024] (molecular function) Relationships: is a type of myosin binding [GO:0017022] Definition: Binding to a class I myosin; myosin I heavy chains are single-headed, possess tails of various lengths, and do not self-associate into bipolar filaments. References: PMID:18344022 Sources: GOC:bf, GOC:mah Subtypes: GO:0032030, myosin I heavy chain binding [GO:0032037]